{
  "gene_symbol": "ORC1",
  "term_id": "GO:0033314",
  "term_label": "mitotic DNA replication checkpoint signaling",
  "gene_name": "Origin recognition complex subunit 1",
  "gene": "UniProtKB:Q13415"
}